{
  "gene": "UniProtKB:P43358",
  "gene_symbol": "MAGEA4",
  "term_label": "histone deacetylase binding",
  "gene_name": "Melanoma-associated antigen 4",
  "term_id": "GO:0042826"
}